{
  "term_label": "cellular response to oxidative stress",
  "term_id": "GO:0034599",
  "gene": "UniProtKB:P00390",
  "gene_symbol": "GSR",
  "gene_name": "Glutathione reductase, mitochondrial"
}